{
  "gene_symbol": "STING1",
  "term_label": "autophagosome",
  "term_id": "GO:0005776",
  "gene_name": "Stimulator of interferon genes protein",
  "gene": "UniProtKB:Q86WV6"
}